{
  "gene": "UniProtKB:Q13191",
  "term_id": "GO:0007165",
  "term_label": "signal transduction",
  "gene_symbol": "CBLB",
  "gene_name": "E3 ubiquitin-protein ligase CBL-B"
}